{
  "gene": "UniProtKB:Q6ZQY7",
  "gene_name": "Putative uncharacterized protein FLJ46792",
  "term_id": "UNKNOWN:0003",
  "term_label": "Unknown cellular component",
  "gene_symbol": "Q6ZQY7"
}